{
  "term_label": "antimicrobial humoral immune response mediated by antimicrobial peptide",
  "gene": "UniProtKB:O00175",
  "gene_name": "C-C motif chemokine 24",
  "term_id": "GO:0061844",
  "gene_symbol": "CCL24"
}